monocarboxylic acid binding [GO:0033293] (molecular function) Definition: Binding to a monocarboxylic acid, any organic acid containing one carboxyl (COOH) group or anion (COO-). Relationships: is a type of carboxylic acid binding [GO:0031406] Sources: GOC:mah Subtypes: retinoic acid binding [GO:0001972], fatty acid binding [GO:0005504], penicillin binding [GO:0008658], GO:0009374, GO:0010013, abscisic acid binding [GO:0010427], bile acid binding [GO:0032052], GO:0032500, ectoine binding [GO:0033294], GO:0033295, galacturonate binding [GO:0048032], salicylic acid binding [GO:1901149], dethiobiotin binding [GO:1901602], GO:1905575